{
  "gene": "UniProtKB:Q7Z4H4",
  "gene_symbol": "ADM2",
  "term_label": "regulation of urine volume",
  "term_id": "GO:0035809",
  "gene_name": "Protein ADM2"
}